{
  "gene_name": "Olfactory receptor 51L1",
  "gene_symbol": "OR51L1",
  "term_label": "Unknown biological process",
  "gene": "UniProtKB:Q8NGJ5",
  "term_id": "UNKNOWN:0002"
}